{
  "gene_name": "Exocyst complex component 6",
  "gene": "UniProtKB:Q8TAG9",
  "gene_symbol": "EXOC6",
  "term_label": "exocytosis",
  "term_id": "GO:0006887"
}